{
  "term_label": "nuclear pore organization",
  "gene_name": "Nucleoporin NUP35",
  "term_id": "GO:0006999",
  "gene": "UniProtKB:Q8NFH5",
  "gene_symbol": "NUP35"
}